negative regulation of mesenchymal cell proliferation [GO:0072201] (biological process) Definition: Any process that decreases the frequency, rate or extent of mesenchymal cell proliferation. A mesenchymal cell is a cell that normally gives rise to other cells that are organized as three-dimensional masses, rather than sheets. Sources: GOC:mtg_kidney_jan10 Relationships: is a type of negative regulation of cell population proliferation [GO:0008285]; is a type of GO:0010464; negatively regulates mesenchymal cell proliferation [GO:0010463] Subtypes: GO:0072200, GO:2000791